regulation of system process [GO:0044057] (biological process) Subtypes: regulation of nervous system process [GO:0031644], GO:0044058, GO:0044060, regulation of excretion [GO:0044062], GO:0044065, regulation of muscle system process [GO:0090257], regulation of renal system process [GO:0098801], regulation of transport across blood-brain barrier [GO:0150200], regulation of blood circulation [GO:1903522], GO:1903814 Sources: GOC:jl Relationships: is_a regulation of multicellular organismal process [GO:0051239]; regulates system process [GO:0003008] Definition: Any process that modulates the frequency, rate or extent of a system process, a multicellular organismal process carried out by any of the organs or tissues in an organ system.